{
  "gene_name": "DDB1- and CUL4-associated factor 8-like protein 1",
  "gene_symbol": "DCAF8L1",
  "gene": "UniProtKB:A6NGE4",
  "term_label": "Unknown molecular function",
  "term_id": "UNKNOWN:0001"
}